{
  "gene_name": "Visual pigment-like receptor peropsin",
  "gene": "UniProtKB:O14718",
  "gene_symbol": "RRH",
  "term_label": "phototransduction",
  "term_id": "GO:0007602"
}